{
  "gene_name": "Deoxyhypusine hydroxylase",
  "term_id": "UNKNOWN:0002",
  "term_label": "Unknown biological process",
  "gene_symbol": "DOHH",
  "gene": "UniProtKB:Q9BU89"
}